pilus assembly [GO:0009297] (biological process) Sources: GOC:dgh, GOC:mcc2, GOC:tb Definition: The assembly from its constituent parts of a pilus, a short filamentous structure of bacterial cell, flagella-like in structure and generally present in many copies. Pili are variously involved in transfer of nucleic acids, adherence to surfaces, and formation of pellicles. Is required for bacterial conjugation, or can play a role in adherence to surfaces (when it is called a fimbrium), and in the formation of pellicles. Also known as: pilus formation, fimbria assembly, fimbriae assembly, fimbrial assembly, fimbrium assembly, fimbria biogenesis, fimbriae biogenesis, fimbrium biogenesis, pilus biogenesis Subtypes: type IV pilus assembly [GO:0043683], GO:0098775, type I pilus assembly [GO:0140623] Relationships: is a type of GO:0030031; is a type of GO:0043711